{
  "gene": "UniProtKB:Q9UI14",
  "term_label": "Unknown molecular function",
  "term_id": "UNKNOWN:0001",
  "gene_symbol": "RABAC1",
  "gene_name": "Prenylated Rab acceptor protein 1"
}